{
  "gene_symbol": "CYP3A7",
  "term_id": "UNKNOWN:0003",
  "term_label": "Unknown cellular component",
  "gene": "UniProtKB:P24462",
  "gene_name": "Cytochrome P450 3A7"
}